{
  "gene_name": "Oxysterol-binding protein-related protein 11",
  "gene_symbol": "OSBPL11",
  "gene": "UniProtKB:Q9BXB4",
  "term_id": "GO:0005794",
  "term_label": "Golgi apparatus"
}